regulation of alternative mRNA splicing, via spliceosome [GO:0000381] (biological process) Relationships: is a type of regulation of mRNA splicing, via spliceosome [GO:0048024]; regulates alternative mRNA splicing, via spliceosome [GO:0000380] Also known as: splice site selection, regulation of alternative nuclear mRNA splicing, via spliceosome Definition: Any process that modulates the frequency, rate or extent of alternative splicing of nuclear mRNAs. Sources: GOC:krc